{
  "gene": "UniProtKB:P16471",
  "gene_name": "Prolactin receptor",
  "term_id": "GO:0004925",
  "term_label": "prolactin receptor activity",
  "gene_symbol": "PRLR"
}